acetoacetate decarboxylase activity [GO:0047602] (molecular function) Definition: Catalysis of the reaction: acetoacetate + H+ = acetone + CO2. Also known as: acetoacetate carboxy-lyase (acetone-forming), acetoacetate carboxy-lyase activity, acetoacetic acid decarboxylase activity Relationships: is a type of carboxy-lyase activity [GO:0016831] Sources: EC:4.1.1.4, RHEA:19729